{
  "gene_name": "Integral membrane protein 2C",
  "gene": "UniProtKB:Q9NQX7",
  "term_label": "negative regulation of amyloid precursor protein biosynthetic process",
  "gene_symbol": "ITM2C",
  "term_id": "GO:0042985"
}